{
  "term_id": "GO:0051642",
  "gene": "UniProtKB:Q8WXH0",
  "gene_symbol": "SYNE2",
  "gene_name": "Nesprin-2",
  "term_label": "centrosome localization"
}